{
  "term_id": "GO:0005634",
  "term_label": "nucleus",
  "gene_symbol": "TBX6",
  "gene_name": "T-box transcription factor TBX6",
  "gene": "UniProtKB:O95947"
}